{
  "gene_name": "Fibroblast growth factor 16",
  "term_id": "GO:0030334",
  "gene": "UniProtKB:O43320",
  "gene_symbol": "FGF16",
  "term_label": "regulation of cell migration"
}